{
  "gene_name": "Cell adhesion molecule 4",
  "gene_symbol": "CADM4",
  "term_id": "GO:0061041",
  "gene": "UniProtKB:Q8NFZ8",
  "term_label": "regulation of wound healing"
}